{
  "gene_symbol": "SPIN1",
  "term_label": "nucleoplasm",
  "gene": "UniProtKB:Q9Y657",
  "term_id": "GO:0005654",
  "gene_name": "Spindlin-1"
}